positive regulation of phosphatidylinositol 3-kinase/protein kinase B signal transduction [GO:0051897] (biological process) Also known as: positive regulation of PI3K-PKB/Akt pathway, positive regulation of PI3K/Akt signal transduction, positive regulation of PI3K/PKB signal transduction, positive regulation of phosphatidylinositol 3-kinase signaling/protein kinase B signal transduction, activation of protein kinase B signaling cascade, stimulation of protein kinase B signaling cascade, positive regulation of AKT signaling cascade, positive regulation of AKT signalling cascade, positive regulation of PKB signaling cascade, positive regulation of PKB signalling cascade, positive regulation of protein kinase B signaling, positive regulation of protein kinase B signaling cascade, positive regulation of protein kinase B signalling cascade, up regulation of protein kinase B signaling cascade, up-regulation of protein kinase B signaling cascade, upregulation of protein kinase B signaling cascade Relationships: is a type of regulation of phosphatidylinositol 3-kinase/protein kinase B signal transduction [GO:0051896]; is a type of positive regulation of intracellular signal transduction [GO:1902533]; positively regulates phosphatidylinositol 3-kinase/protein kinase B signal transduction [GO:0043491] Sources: GOC:ai Definition: Any process that activates or increases the frequency, rate or extent of phosphatidylinositol 3-kinase/protein kinase B signal transduction.